{
  "gene": "UniProtKB:Q9Y584",
  "gene_name": "Mitochondrial import inner membrane translocase subunit Tim22",
  "term_label": "mitochondrion targeting sequence binding",
  "term_id": "GO:0030943",
  "gene_symbol": "TIMM22"
}